{
  "term_id": "GO:0004322",
  "gene": "UniProtKB:Q9BQS7",
  "term_label": "ferroxidase activity",
  "gene_symbol": "HEPH",
  "gene_name": "Hephaestin"
}